{
  "term_label": "mitotic G2 DNA damage checkpoint signaling",
  "gene_name": "Claspin",
  "gene_symbol": "CLSPN",
  "gene": "UniProtKB:Q9HAW4",
  "term_id": "GO:0007095"
}